{
  "term_label": "oxidoreductase activity",
  "gene_name": "Very-long-chain 3-oxoacyl-CoA reductase",
  "gene": "UniProtKB:Q53GQ0",
  "gene_symbol": "HSD17B12",
  "term_id": "GO:0016491"
}